{
  "gene_symbol": "TMPRSS5",
  "term_id": "GO:0008236",
  "term_label": "serine-type peptidase activity",
  "gene_name": "Transmembrane protease serine 5",
  "gene": "UniProtKB:Q9H3S3"
}